peptide cross-linking [GO:0018149] (biological process) Definition: The formation of a covalent cross-link between or within protein chains. Sources: GOC:jsg Relationships: is_a protein modification process [GO:0036211] Subtypes: isopeptide cross-linking [GO:0018262], peptide cross-linking via L-cystine [GO:0018316]